negative regulation of intralumenal vesicle formation [GO:1905366] (biological process) Also known as: down regulation of endosome membrane budding, down regulation of intralumenal vesicle formation, down-regulation of endosome membrane budding, down-regulation of intralumenal vesicle formation, downregulation of endosome membrane budding, downregulation of intralumenal vesicle formation, negative regulation of endosome membrane budding, inhibition of endosome membrane budding, inhibition of intralumenal vesicle formation References: PMID:26911690 Sources: GOC:PARL, GOC:TermGenie, GOC:bc, GO_REF:0000058 Definition: Any process that stops, prevents or reduces the frequency, rate or extent of intralumenal vesicle formation. Relationships: is a type of negative regulation of transport [GO:0051051]; is a type of negative regulation of endosome organization [GO:1904979]; is a type of regulation of intralumenal vesicle formation [GO:1905365]; negatively regulates intralumenal vesicle formation [GO:0070676]